{
  "gene_symbol": "MMP27",
  "gene_name": "Matrix metalloproteinase-27",
  "term_label": "metalloendopeptidase activity",
  "gene": "UniProtKB:Q9H306",
  "term_id": "GO:0004222"
}